{
  "term_label": "axon",
  "gene_name": "Synaptotagmin-1",
  "gene_symbol": "SYT1",
  "gene": "UniProtKB:P21579",
  "term_id": "GO:0030424"
}